UGC codon-amino acid adaptor activity [GO:0033414] (molecular function) Also known as: TGC codon-amino acid adaptor activity, cysteine tRNA Relationships: is a type of GO:0030533 Definition: A triplet codon-amino acid adaptor activity that recognizes a UGC codon. Note: Note that in the standard genetic code, TGC codes for cysteine. Sources: GOC:mah